{
  "gene_name": "Transmembrane and coiled-coil domain-containing protein 4",
  "gene": "UniProtKB:Q5TGY1",
  "term_label": "Unknown biological process",
  "gene_symbol": "TMCO4",
  "term_id": "UNKNOWN:0002"
}